{
  "gene_name": "Stromelysin-3",
  "term_label": "metalloendopeptidase activity",
  "term_id": "GO:0004222",
  "gene": "UniProtKB:P24347",
  "gene_symbol": "MMP11"
}